ganglioside GM1 binding [GO:1905573] (molecular function) Relationships: is a type of GO:0031406; is a type of ganglioside binding [GO:0035594] References: PMID:1454804 Sources: GOC:TermGenie, GO_REF:0000067 Definition: Binding to ganglioside GM1.